{
  "term_id": "UNKNOWN:0003",
  "gene_name": "Chordin-like protein 1",
  "gene_symbol": "CHRDL1",
  "gene": "UniProtKB:Q9BU40",
  "term_label": "Unknown cellular component"
}